{
  "term_label": "cytoplasm",
  "term_id": "GO:0005737",
  "gene_name": "Ornithine decarboxylase antizyme 2",
  "gene_symbol": "OAZ2",
  "gene": "UniProtKB:O95190"
}